{
  "term_id": "GO:0000977",
  "term_label": "RNA polymerase II transcription regulatory region sequence-specific DNA binding",
  "gene": "UniProtKB:Q14190",
  "gene_symbol": "SIM2",
  "gene_name": "Single-minded homolog 2"
}